{
  "gene": "UniProtKB:Q6P474",
  "term_label": "Unknown molecular function",
  "term_id": "UNKNOWN:0001",
  "gene_name": "Putative pyridoxal-dependent decarboxylase domain-containing protein 2",
  "gene_symbol": "PDXDC2P"
}